{
  "gene": "UniProtKB:P22760",
  "term_id": "GO:0004806",
  "term_label": "triacylglycerol lipase activity",
  "gene_symbol": "AADAC",
  "gene_name": "Arylacetamide deacetylase"
}